{
  "term_id": "GO:0015485",
  "gene_symbol": "OSBPL7",
  "term_label": "cholesterol binding",
  "gene": "UniProtKB:Q9BZF2",
  "gene_name": "Oxysterol-binding protein-related protein 7"
}